{
  "term_label": "Unknown molecular function",
  "gene_symbol": "THAP10",
  "gene_name": "THAP domain-containing protein 10",
  "term_id": "UNKNOWN:0001",
  "gene": "UniProtKB:Q9P2Z0"
}